mating projection septin band [GO:0032162] (cellular component) Definition: A septin band, i.e. a diffuse ring composed of a series of septin bars running parallel to the long axis of the cell, located at the neck of a shmoo (mating projection). Relationships: is a type of septin band [GO:0032158]; is part of GO:0005937 References: PMID:16151244 Sources: GOC:krc, GOC:mah